ATF4-CREB1 transcription factor complex [GO:1990589] (cellular component) Definition: Transcription factor complex consisting of ATF4 and CREB1 subunits that is capable of binding to cAMP response element (CRE) (consensus: 5'-GTGACGT[AC][AG]-3') as part of the positive regulation of transcription. Regulatory targets include the GRP78 (HSPA5) promoter in humans, whose activation by this complex is part of the ER stress response pathway. Relationships: is a type of RNA polymerase II transcription regulator complex [GO:0090575] References: PMID:12871976 Sources: GOC:bhm